positive regulation of lymphocyte differentiation [GO:0045621] (biological process) Definition: Any process that activates or increases the frequency, rate or extent of lymphocyte differentiation. Also known as: up regulation of lymphocyte differentiation, up-regulation of lymphocyte differentiation, upregulation of lymphocyte differentiation, activation of lymphocyte differentiation, stimulation of lymphocyte differentiation, positive regulation of lymphocyte development Sources: GOC:go_curators Note: Note that immunologists typically use the word 'development' to refer to cells of B or T cell lineages undergoing the process that GO describes as 'cell differentiation'. Relationships: is a type of GO:0045619; is a type of positive regulation of lymphocyte activation [GO:0051251]; is a type of GO:1902107; positively regulates lymphocyte differentiation [GO:0030098] Subtypes: positive regulation of natural killer cell differentiation [GO:0032825], positive regulation of B cell differentiation [GO:0045579], positive regulation of T cell differentiation [GO:0045582]